{
  "gene": "UniProtKB:O43913",
  "term_label": "DNA replication initiation",
  "gene_name": "Origin recognition complex subunit 5",
  "gene_symbol": "ORC5",
  "term_id": "GO:0006270"
}